{
  "gene_name": "Palmitoyltransferase ZDHHC7",
  "gene_symbol": "ZDHHC7",
  "gene": "UniProtKB:Q9NXF8",
  "term_label": "Golgi apparatus",
  "term_id": "GO:0005794"
}